{
  "term_id": "UNKNOWN:0003",
  "term_label": "Unknown cellular component",
  "gene_name": "V-type proton ATPase subunit H",
  "gene": "UniProtKB:Q9UI12",
  "gene_symbol": "ATP6V1H"
}